{
  "term_id": "GO:0042622",
  "gene_name": "Photoreceptor disk component PRCD",
  "gene": "UniProtKB:Q00LT1",
  "gene_symbol": "PRCD",
  "term_label": "photoreceptor outer segment membrane"
}